{
  "gene_name": "Olfactory receptor 2AT4",
  "term_label": "olfactory receptor activity",
  "term_id": "GO:0004984",
  "gene_symbol": "OR2AT4",
  "gene": "UniProtKB:A6NND4"
}